{
  "term_label": "olfactory receptor activity",
  "term_id": "GO:0004984",
  "gene_symbol": "OR10C1",
  "gene": "UniProtKB:Q96KK4",
  "gene_name": "Olfactory receptor 10C1"
}